{
  "gene_symbol": "LTC4S",
  "gene_name": "Leukotriene C4 synthase",
  "gene": "UniProtKB:Q16873",
  "term_id": "GO:0019370",
  "term_label": "leukotriene biosynthetic process"
}